meiotic G2 phase [GO:0051331] (biological process) Also known as: G2 phase of meiotic cell cycle Relationships: is a type of GO:0051319; is part of GO:0051328 Definition: The cell cycle 'gap' phase which is the interval between the completion of DNA synthesis and the beginning of DNA segregation by meiosis. Sources: GOC:mtg_cell_cycle Note: Note that this term should not be used for direct annotation. If you are trying to make an annotation to x phase, it is likely that the correct annotation is 'regulation of x/y phase transition' or to a process which occurs during the reported phase (i.e mitotic DNA replication for mitotic S-phase). To capture the phase when a specific location or process is observed, the phase term can be used in an annotation extension (PMID:24885854) applied to a cellular component term (with the relation exists_during) or a biological process term (with the relation happens_during).